positive regulation of respiratory burst involved in inflammatory response [GO:0060265] (biological process) Also known as: positive regulation of respiratory burst involved in acute inflammatory response Relationships: is a type of positive regulation of immune effector process [GO:0002699]; is a type of GO:0045089; is a type of GO:0050729; is a type of positive regulation of multicellular organismal process [GO:0051240]; is a type of regulation of respiratory burst involved in inflammatory response [GO:0060264]; is a type of positive regulation of respiratory burst [GO:0060267]; positively regulates respiratory burst involved in inflammatory response [GO:0002536] Sources: GOC:BHF, GOC:dph, GOC:tb Definition: Any process that increases the rate, frequency or extent of a phase of elevated metabolic activity, during which oxygen consumption increases made as a defense response ; this leads to the production, by an NADH dependent system, of hydrogen peroxide (H2O2), superoxide anions and hydroxyl radicals.